{
  "gene_symbol": "ZNF778",
  "term_id": "GO:0005634",
  "gene": "UniProtKB:Q96MU6",
  "term_label": "nucleus",
  "gene_name": "Zinc finger protein 778"
}